{
  "gene_symbol": "CFAP74",
  "term_id": "UNKNOWN:0001",
  "gene_name": "Cilia- and flagella-associated protein 74",
  "term_label": "Unknown molecular function",
  "gene": "UniProtKB:Q9C0B2"
}